AAC codon-amino acid adaptor activity [GO:0033442] (molecular function) Definition: A triplet codon-amino acid adaptor activity that recognizes an AAC codon. Note: Note that in the standard genetic code, AAC codes for asparagine. Relationships: is a type of triplet codon-amino acid adaptor activity [GO:0030533] Also known as: asparagine tRNA Sources: GOC:mah